{
  "gene_symbol": "LDLRAP1",
  "term_id": "UNKNOWN:0002",
  "gene_name": "Low density lipoprotein receptor adapter protein 1",
  "gene": "UniProtKB:Q5SW96",
  "term_label": "Unknown biological process"
}